{
  "term_id": "GO:0004222",
  "term_label": "metalloendopeptidase activity",
  "gene_symbol": "ADAMTS16",
  "gene": "UniProtKB:Q8TE57",
  "gene_name": "A disintegrin and metalloproteinase with thrombospondin motifs 16"
}